{
  "gene_symbol": "OR51I1",
  "term_id": "GO:0004984",
  "term_label": "olfactory receptor activity",
  "gene": "UniProtKB:Q9H343",
  "gene_name": "Olfactory receptor 51I1"
}